{
  "gene_name": "Ankyrin repeat domain-containing protein 39",
  "term_id": "UNKNOWN:0003",
  "gene": "UniProtKB:Q53RE8",
  "gene_symbol": "ANKRD39",
  "term_label": "Unknown cellular component"
}